{
  "gene_symbol": "DCUN1D1",
  "gene_name": "DCN1-like protein 1",
  "term_label": "ubiquitin ligase complex",
  "gene": "UniProtKB:Q96GG9",
  "term_id": "GO:0000151"
}